{
  "gene": "UniProtKB:Q9H8K7",
  "term_id": "UNKNOWN:0002",
  "gene_symbol": "PAAT",
  "term_label": "Unknown biological process",
  "gene_name": "ATPase PAAT"
}